presynaptic periactive zone [GO:0036062] (CC) Also known as: periactive zone, pre-synaptic periactive zone Definition: A region that surrounds the active zone of the presynaptic plasma membrane, and is specialized for the control of synaptic development. Relationships: is a type of GO:0097060; is part of presynaptic membrane [GO:0042734] References: PMID:10976048, PMID:18439406 Sources: GOC:sart